chloroplast stromal thylakoid [GO:0009533] (CC) Sources: ISBN:0943088399 Definition: Unstacked thylakoids that connect the grana stacks through the stroma. Relationships: is a type of GO:0009534; is part of GO:0009570